{
  "gene": "UniProtKB:Q8WVJ9",
  "gene_symbol": "TWIST2",
  "gene_name": "Twist-related protein 2",
  "term_id": "UNKNOWN:0003",
  "term_label": "Unknown cellular component"
}